{
  "gene_name": "Epididymal-specific lipocalin-10",
  "gene": "UniProtKB:Q6JVE6",
  "term_label": "Unknown cellular component",
  "gene_symbol": "LCN10",
  "term_id": "UNKNOWN:0003"
}